histone H3K27 trimethyltransferase activity [GO:0140951] (molecular function) Relationships: is a type of histone H3K27 methyltransferase activity [GO:0046976] Note: Comment: Note that the residue position corresponds to the canonical human H3 histone (UniProtKB:P84243); this residue is conserved across all eukaryotes. Residue 1 is the first residue following removal of the initiating Methionine (Met). Note that each histone is encoded by multiple genes, and sequences may vary across different genes within an organism. Sources: RHEA:60292 Also known as: histone H3-K27 trimethylation, histone H3K27 trimethylation, histone H3-K27 trimethylase activity, histone H3K27 mono/di/trimethylase activity, histone H3K27 trimethylase activity, histone lysine N-trimethyltransferase activity (H3-K27 specific) Definition: Catalysis of the reaction: L-lysyl27-[histone H3] + 3 S-adenosyl-L-methionine = 3 H+ + N6,N6,N6-trimethyl-L-lysyl27-[histone H3] + 3 S-adenosyl-L-homocysteine. This reaction is the successive addition of three methyl groups to the unmethylated lysine residue at position 27 of histone H3, producing histone H3K27me3.